{
  "term_id": "GO:0043161",
  "gene_symbol": "FBXW7",
  "gene": "UniProtKB:Q969H0",
  "gene_name": "F-box_WD repeat-containing protein 7",
  "term_label": "proteasome-mediated ubiquitin-dependent protein catabolic process"
}